{
  "gene_name": "RNA-splicing ligase RtcB homolog",
  "gene_symbol": "RTCB",
  "gene": "UniProtKB:Q9Y3I0",
  "term_id": "GO:0006388",
  "term_label": "tRNA splicing, via endonucleolytic cleavage and ligation"
}